{
  "term_label": "Unknown molecular function",
  "term_id": "UNKNOWN:0001",
  "gene_symbol": "P3R3URF",
  "gene": "UniProtKB:A0A087WWA1",
  "gene_name": "PIK3R3 upstream open reading frame protein"
}